{
  "gene": "UniProtKB:Q5T871",
  "term_label": "Unknown molecular function",
  "term_id": "UNKNOWN:0001",
  "gene_symbol": "LELP1",
  "gene_name": "Late cornified envelope-like proline-rich protein 1"
}